{
  "gene_name": "Polyadenylate-binding protein 3",
  "gene": "UniProtKB:Q9H361",
  "gene_symbol": "PABPC3",
  "term_label": "cytosol",
  "term_id": "GO:0005829"
}